{
  "gene_name": "Vesicle transport through interaction with t-SNAREs homolog 1B",
  "gene": "UniProtKB:Q9UEU0",
  "gene_symbol": "VTI1B",
  "term_label": "SNAP receptor activity",
  "term_id": "GO:0005484"
}